conditioned place preference [GO:1990708] (biological process) Definition: The associative learning process by which an animal learns and remembers an association between a neutral, unchanging environment and a putatively rewarding, internal state produced by a xenobiotic or drug. Relationships: is a type of associative learning [GO:0008306] References: PMID:21549821